polyubiquitin modification-dependent protein binding [GO:0031593] (molecular function) Definition: Binding to a protein upon poly-ubiquitination of the target protein. Sources: GOC:pg Subtypes: K48-linked polyubiquitin modification-dependent protein binding [GO:0036435], GO:0070530, K11-linked polyubiquitin modification-dependent protein binding [GO:0071795], K6-linked polyubiquitin modification-dependent protein binding [GO:0071796] Relationships: is_a modification-dependent protein binding [GO:0140030]